{
  "gene": "UniProtKB:P46736",
  "term_label": "BRCA1-A complex",
  "term_id": "GO:0070531",
  "gene_symbol": "BRCC3",
  "gene_name": "Lys-63-specific deubiquitinase BRCC36"
}